{
  "gene_symbol": "SMAD3",
  "term_label": "SMAD protein signal transduction",
  "gene": "UniProtKB:P84022",
  "term_id": "GO:0060395",
  "gene_name": "Mothers against decapentaplegic homolog 3"
}